{
  "term_label": "response to nicotine",
  "gene_symbol": "CHRNA5",
  "term_id": "GO:0035094",
  "gene": "UniProtKB:P30532",
  "gene_name": "Neuronal acetylcholine receptor subunit alpha-5"
}